{
  "term_label": "DNA-binding transcription repressor activity, RNA polymerase II-specific",
  "term_id": "GO:0001227",
  "gene": "UniProtKB:Q9HC78",
  "gene_name": "Zinc finger and BTB domain-containing protein 20",
  "gene_symbol": "ZBTB20"
}